negative regulation of vasculature development involved in avascular cornea development in camera-type eye [GO:1901346] (biological process) Definition: Any negative regulation of vasculature development that is involved in developing an avascular cornea of a camera-type eye. Also known as: down regulation of vasculature development involved in avascular cornea development, down regulation of vasculature development involved in avascular cornea development in camera-type eye, down-regulation of vasculature development involved in avascular cornea development, down-regulation of vasculature development involved in avascular cornea development in camera-type eye, downregulation of vasculature development involved in avascular cornea development, downregulation of vasculature development involved in avascular cornea development in camera-type eye, negative regulation of vasculature development involved in avascular cornea development, inhibition of vasculature development involved in avascular cornea development, inhibition of vasculature development involved in avascular cornea development in camera-type eye, down regulation of vascular system development involved in avascular cornea development, down regulation of vascular system development involved in avascular cornea development in camera-type eye, down-regulation of vascular system development involved in avascular cornea development, down-regulation of vascular system development involved in avascular cornea development in camera-type eye, downregulation of vascular system development involved in avascular cornea development, downregulation of vascular system development involved in avascular cornea development in camera-type eye, inhibition of vascular system development involved in avascular cornea development, inhibition of vascular system development involved in avascular cornea development in camera-type eye, negative regulation of vascular system development involved in avascular cornea development, negative regulation of vascular system development involved in avascular cornea development in camera-type eye References: PMID:16849433, PMID:17051153 Sources: GOC:TermGenie, GOC:uh Relationships: is a type of negative regulation of vasculature development [GO:1901343]; is part of GO:0036331